{
  "gene_name": "Protein-cysteine N-palmitoyltransferase HHAT-like protein",
  "gene_symbol": "HHATL",
  "term_label": "Unknown molecular function",
  "term_id": "UNKNOWN:0001",
  "gene": "UniProtKB:Q9HCP6"
}